{
  "term_id": "UNKNOWN:0003",
  "gene_name": "Zinc finger E-box-binding homeobox 1",
  "gene_symbol": "ZEB1",
  "term_label": "Unknown cellular component",
  "gene": "UniProtKB:P37275"
}